{
  "gene_symbol": "ZNF101",
  "gene_name": "Zinc finger protein 101",
  "term_label": "regulation of transcription by RNA polymerase II",
  "term_id": "GO:0006357",
  "gene": "UniProtKB:Q8IZC7"
}